negative regulation of encysted zoospore germination [GO:0075229] (biological process) Definition: Any process that stops, prevents, or reduces the frequency, rate or extent of encysted zoospore germination. Sources: GOC:pamgo_curators Also known as: negative regulation of encysted zoospore germination on or near host Relationships: is a type of regulation of encysted zoospore germination [GO:0075227]; is a type of GO:1904360; negatively regulates encysted zoospore germination [GO:0075226]